positive regulation of mesenchymal cell proliferation [GO:0002053] (biological process) Subtypes: positive regulation of metanephric cap mesenchymal cell proliferation [GO:0090096], positive regulation of mesenchymal cell proliferation involved in ureter development [GO:2000729], positive regulation of mesenchymal cell proliferation involved in lung development [GO:2000792] Definition: The process of activating or increasing the rate or extent of mesenchymal cell proliferation. Mesenchymal cells are loosely organized embryonic cells. Relationships: is a type of positive regulation of cell population proliferation [GO:0008284]; is a type of regulation of mesenchymal cell proliferation [GO:0010464]; positively regulates GO:0010463 Sources: GOC:dph Also known as: up regulation of mesenchymal cell proliferation, up-regulation of mesenchymal cell proliferation, upregulation of mesenchymal cell proliferation, activation of mesenchymal cell proliferation, stimulation of mesenchymal cell proliferation